MacAB-TolC complex [GO:1990196] (cellular component) Also known as: macrolide transporter MacAB-TolC complex Relationships: is a type of macrolide transmembrane transporter complex [GO:1990195] References: PMID:10879525, PMID:18955484, PMID:19254725 Sources: GOC:bhm Definition: The MacAB-TolC complex is a macrolide transporter complex found in E.coli and related gram-negative bacteria. Its transport activity is specific to macrolide compounds containing 14- and 15-membered lactones. It consists of the dimeric inner membrane ATPase MacB, the hexameric, periplasmic membrane fusion protein MacA and the trimeric outer membrane factor TolC.